{
  "gene": "UniProtKB:Q86YQ2",
  "gene_name": "Putative BPIFA4P protein",
  "term_label": "Unknown molecular function",
  "gene_symbol": "BPIFA4P",
  "term_id": "UNKNOWN:0001"
}